{
  "gene_name": "Leukotriene A-4 hydrolase",
  "term_label": "leukotriene-A4 hydrolase activity",
  "gene_symbol": "LTA4H",
  "gene": "UniProtKB:P09960",
  "term_id": "GO:0004463"
}